{
  "term_label": "nuclear speck",
  "term_id": "GO:0016607",
  "gene_name": "Serine_arginine-rich splicing factor 6",
  "gene_symbol": "SRSF6",
  "gene": "UniProtKB:Q13247"
}